{
  "gene_name": "Homeobox protein CDX-4",
  "gene_symbol": "CDX4",
  "term_id": "GO:0009948",
  "gene": "UniProtKB:O14627",
  "term_label": "anterior/posterior axis specification"
}